{
  "gene": "UniProtKB:Q8N2N9",
  "gene_name": "Ankyrin repeat domain-containing protein 36B",
  "term_id": "UNKNOWN:0002",
  "term_label": "Unknown biological process",
  "gene_symbol": "ANKRD36B"
}